{
  "gene_name": "Ankyrin repeat domain-containing protein 29",
  "gene": "UniProtKB:Q8N6D5",
  "gene_symbol": "ANKRD29",
  "term_id": "UNKNOWN:0001",
  "term_label": "Unknown molecular function"
}